{
  "term_id": "GO:0046403",
  "gene": "UniProtKB:Q96T60",
  "term_label": "polynucleotide 3'-phosphatase activity",
  "gene_symbol": "PNKP",
  "gene_name": "Bifunctional polynucleotide phosphatase_kinase"
}